{
  "gene_symbol": "RGS7BP",
  "term_id": "GO:0098794",
  "gene_name": "Regulator of G-protein signaling 7-binding protein",
  "term_label": "postsynapse",
  "gene": "UniProtKB:Q6MZT1"
}